retinol transmembrane transporter activity [GO:0034632] (molecular function) Relationships: is a type of alcohol transmembrane transporter activity [GO:0015665]; is a type of vitamin transmembrane transporter activity [GO:0090482]; is a type of lipid transmembrane transporter activity [GO:0170055]; is part of retinol transport [GO:0034633] Definition: Enables the transfer of retinol from one side of a membrane to the other. Retinol is vitamin A1, 2,6,6-trimethyl-1-(9'-hydroxy-3',7'-dimethylnona-1',3',5',7'-tetraenyl)cyclohex-1-ene, one of the three components that makes up vitamin A. Sources: GOC:BHF, GOC:mah, GOC:vk Also known as: vitamin A1 transporter activity, retinol transporter activity